ether lipid biosynthetic process [GO:0008611] (biological process) Subtypes: platelet activating factor biosynthetic process [GO:0006663] Definition: The chemical reactions and pathways resulting in the formation of ether lipids, lipids that contain (normally) one lipid alcohol in ether linkage to one of the carbon atoms (normally C-1) of glycerol. Also known as: ether lipid anabolism, ether lipid biosynthesis, ether lipid formation, ether lipid synthesis, plasmalogen biosynthetic process References: PMID:15337120 Sources: GOC:ma, ISBN:0198547684 Relationships: is a type of lipid biosynthetic process [GO:0008610]; is a type of ether lipid metabolic process [GO:0046485]; is a type of GO:0046504